{
  "term_id": "GO:0002682",
  "term_label": "regulation of immune system process",
  "gene_name": "Carcinoembryonic antigen-related cell adhesion molecule 1",
  "gene": "UniProtKB:P13688",
  "gene_symbol": "CEACAM1"
}